{
  "gene_symbol": "ERICH2",
  "term_label": "Unknown biological process",
  "gene_name": "Glutamate-rich protein 2",
  "gene": "UniProtKB:A1L162",
  "term_id": "UNKNOWN:0002"
}